establishment of epithelial cell polarity [GO:0090162] (biological process) Subtypes: GO:0045198, establishment of epithelial cell planar polarity [GO:0090163] Relationships: is a type of establishment of cell polarity [GO:0030010] Definition: The specification and formation of anisotropic intracellular organization of an epithelial cell. Sources: GOC:ascb_2009, GOC:dph, GOC:tb